Hrd1p ubiquitin ligase ERAD-L complex [GO:0000839] (cellular component) Relationships: is a type of Hrd1p ubiquitin ligase complex [GO:0000836] References: PMID:16873065, PMID:16873066 Sources: GOC:elh Definition: A multiprotein complex that recognizes and ubiquitinates proteins with misfolded luminal domains during ER-associated protein degradation (ERAD). In S. cerevisiae, this complex contains the ubiquitin ligase Hrd1p.